{
  "gene_symbol": "KARS1",
  "term_label": "positive regulation of macrophage activation",
  "term_id": "GO:0043032",
  "gene": "UniProtKB:Q15046",
  "gene_name": "Lysine--tRNA ligase"
}